inhibin-betaglycan-ActRII complex [GO:0034673] (cellular component) Definition: A protein complex that consists of inhibin, type III transforming growth factor beta receptor (also known as betaglycan), and the type II activin receptor ActRII. The complex is thought to negatively regulate the activity of activin B. Relationships: is_a plasma membrane protein complex [GO:0098797] References: PMID:10746731 Sources: GOC:BHF